{
  "gene_symbol": "LIPM",
  "term_id": "UNKNOWN:0003",
  "gene_name": "Lipase member M",
  "gene": "UniProtKB:Q5VYY2",
  "term_label": "Unknown cellular component"
}